negative regulation of carbohydrate metabolic process [GO:0045912] (biological process) Relationships: is a type of GO:0006109; is a type of GO:0009892; negatively regulates carbohydrate metabolic process [GO:0005975] Sources: GOC:go_curators Also known as: down regulation of carbohydrate metabolic process, down-regulation of carbohydrate metabolic process, downregulation of carbohydrate metabolic process, negative regulation of carbohydrate metabolism, inhibition of carbohydrate metabolic process Definition: Any process that stops, prevents, or reduces the frequency, rate or extent of the chemical reactions and pathways involving carbohydrate. Subtypes: GO:0010323, negative regulation of inositol phosphate biosynthetic process [GO:0010920], negative regulation of gluconeogenesis [GO:0045721], negative regulation of glycolytic process [GO:0045820], GO:0060636, negative regulation of glycogen metabolic process [GO:0070874], negative regulation of reductive pentose-phosphate cycle [GO:0080153], negative regulation of raffinose biosynthetic process [GO:1900092], negative regulation of hyaluronan biosynthetic process [GO:1900126], negative regulation of cellobiose catabolic process [GO:1900283], negative regulation of xylose catabolic process to ethanol [GO:1900516], negative regulation of lactose biosynthetic process [GO:1903535], negative regulation of glucose catabolic process to lactate via pyruvate [GO:1904024], GO:2000083, negative regulation of glyoxylate cycle [GO:2000875], GO:2000882, GO:2000907, GO:2000913, negative regulation of cellodextrin catabolic process [GO:2000928], GO:2000937, negative regulation of cyclodextrin catabolic process [GO:2000958], negative regulation of cellooligosaccharide catabolic process [GO:2000964], negative regulation of cell wall polysaccharide catabolic process [GO:2000967], negative regulation of hemicellulose catabolic process [GO:2000989], GO:2000992, negative regulation of cellulose catabolic process [GO:2000998], negative regulation of pectin catabolic process [GO:2001004], GO:2001007, negative regulation of glycolytic fermentation to ethanol [GO:2001155], negative regulation of starch biosynthetic process [GO:7770012]